{
  "term_id": "GO:0005737",
  "gene_name": "Tumor protein D55",
  "term_label": "cytoplasm",
  "gene_symbol": "TPD52L3",
  "gene": "UniProtKB:Q96J77"
}